{
  "gene_name": "Testis-expressed protein 35",
  "gene": "UniProtKB:Q5T0J7",
  "term_label": "Unknown biological process",
  "term_id": "UNKNOWN:0002",
  "gene_symbol": "TEX35"
}